polytene chromosome band [GO:0005704] (cellular component) Definition: A stretch of densely packed chromatin along the polytene chromosome, visible as a morphologically distinct band. References: PMID:11361342 Sources: GOC:bf Relationships: is_a chromosomal region [GO:0098687]; is part of GO:0005700